{
  "term_id": "UNKNOWN:0001",
  "term_label": "Unknown molecular function",
  "gene_symbol": "IGLV10-54",
  "gene_name": "Immunoglobulin lambda variable 10-54",
  "gene": "UniProtKB:A0A075B6I4"
}